regulation of protein localization to medial cortical node [GO:0120046] (biological process) References: PMID:19474789 Subtypes: GO:0120047 Definition: Any process that modulates the frequency, rate or extent of protein localization to a medial cortical node. Relationships: is a type of regulation of protein localization to medial cortex [GO:0106011]; regulates protein localization to medial cortical node [GO:1902577]